{
  "gene": "UniProtKB:P0CG12",
  "gene_name": "Decreased expression in renal and prostate cancer protein",
  "gene_symbol": "DERPC",
  "term_id": "UNKNOWN:0002",
  "term_label": "Unknown biological process"
}